{
  "gene": "UniProtKB:Q5VZK9",
  "term_label": "Unknown molecular function",
  "term_id": "UNKNOWN:0001",
  "gene_name": "F-actin-uncapping protein LRRC16A",
  "gene_symbol": "CARMIL1"
}